{
  "term_label": "dendrite",
  "gene_symbol": "STRN3",
  "term_id": "GO:0030425",
  "gene": "UniProtKB:Q13033",
  "gene_name": "Striatin-3"
}